{
  "gene_symbol": "PSMB11",
  "term_label": "proteasome-mediated ubiquitin-dependent protein catabolic process",
  "term_id": "GO:0043161",
  "gene_name": "Proteasome subunit beta type-11",
  "gene": "UniProtKB:A5LHX3"
}